negative regulation of pyrimidine nucleobase metabolic process [GO:0045984] (biological process) Also known as: down regulation of pyrimidine base metabolic process, down-regulation of pyrimidine base metabolic process, downregulation of pyrimidine base metabolic process, negative regulation of pyrimidine base metabolic process, negative regulation of pyrimidine base metabolism, inhibition of pyrimidine base metabolic process Sources: GOC:go_curators Definition: Any process that stops, prevents, or reduces the frequency, rate or extent of the chemical reactions and pathways involving pyrimidine nucleobases. Relationships: is a type of negative regulation of nucleobase-containing compound metabolic process [GO:0045934]; is a type of negative regulation of small molecule metabolic process [GO:0062014]; negatively regulates pyrimidine nucleobase metabolic process [GO:0006206]